{
  "term_label": "Unknown molecular function",
  "gene_name": "Protein GAPT",
  "gene_symbol": "GAPT",
  "gene": "UniProtKB:Q8N292",
  "term_id": "UNKNOWN:0001"
}